{
  "term_id": "GO:0005634",
  "gene_symbol": "S100PBP",
  "gene_name": "S100P-binding protein",
  "gene": "UniProtKB:Q96BU1",
  "term_label": "nucleus"
}